{
  "term_label": "cell surface receptor protein tyrosine kinase signaling pathway",
  "term_id": "GO:0007169",
  "gene_name": "Lymphocyte cytosolic protein 2",
  "gene_symbol": "LCP2",
  "gene": "UniProtKB:Q13094"
}